{
  "term_id": "GO:0005737",
  "gene_name": "Serine_threonine-protein kinase haspin",
  "term_label": "cytoplasm",
  "gene_symbol": "HASPIN",
  "gene": "UniProtKB:Q8TF76"
}